{
  "gene": "UniProtKB:Q9H0E2",
  "gene_symbol": "TOLLIP",
  "term_id": "GO:0006511",
  "term_label": "ubiquitin-dependent protein catabolic process",
  "gene_name": "Toll-interacting protein"
}